{
  "gene_symbol": "PP2D1",
  "term_label": "negative regulation of MAPK cascade",
  "term_id": "GO:0043409",
  "gene_name": "Protein phosphatase 2C-like domain-containing protein 1",
  "gene": "UniProtKB:A8MPX8"
}